{
  "gene_symbol": "CCND3",
  "term_label": "cyclin-dependent protein kinase holoenzyme complex",
  "gene_name": "G1_S-specific cyclin-D3",
  "term_id": "GO:0000307",
  "gene": "UniProtKB:P30281"
}